{
  "term_label": "mRNA binding",
  "term_id": "GO:0003729",
  "gene_name": "Probable ATP-dependent RNA helicase DDX41",
  "gene_symbol": "DDX41",
  "gene": "UniProtKB:Q9UJV9"
}